{
  "term_id": "GO:0032006",
  "gene_name": "Protein FAM83D",
  "term_label": "regulation of TOR signaling",
  "gene_symbol": "FAM83D",
  "gene": "UniProtKB:Q9H4H8"
}